{
  "term_label": "non-membrane spanning protein tyrosine kinase activity",
  "gene_symbol": "TEC",
  "gene_name": "Tyrosine-protein kinase Tec",
  "term_id": "GO:0004715",
  "gene": "UniProtKB:P42680"
}